{
  "gene": "UniProtKB:P40227",
  "term_label": "unfolded protein binding",
  "gene_name": "T-complex protein 1 subunit zeta",
  "term_id": "GO:0051082",
  "gene_symbol": "CCT6A"
}